{
  "gene_symbol": "SYDE1",
  "term_id": "GO:0046578",
  "gene_name": "Rho GTPase-activating protein SYDE1",
  "gene": "UniProtKB:Q6ZW31",
  "term_label": "regulation of Ras protein signal transduction"
}